steroid dehydrogenase activity, acting on the CH-OH group of donors, NAD or NADP as acceptor [GO:0033764] (molecular function) Relationships: is a type of steroid dehydrogenase activity [GO:0016229]; is a type of oxidoreductase activity, acting on the CH-OH group of donors, NAD or NADP as acceptor [GO:0016616] Sources: GOC:mah Definition: Catalysis of an oxidation-reduction (redox) reaction in which a CH-OH group acts as a hydrogen or electron donor and reduces NAD+ or NADP, and in which one substrate is a sterol derivative. Subtypes: GO:0000252, 3-beta-hydroxysteroid 3-dehydrogenase (NADP+) activity [GO:0000253], 3-beta-hydroxy-Delta5-steroid dehydrogenase (NAD+) activity [GO:0003854], estradiol 17-beta-dehydrogenase [NAD(P)+] activity [GO:0004303], GO:0008709, 3-beta-hydroxy-5-beta-steroid dehydrogenase (NADP+) activity [GO:0033703], GO:0033704, 17-beta-hydroxysteroid dehydrogenase (NAD+) activity [GO:0044594], 17-alpha,20-alpha-dihydroxypregn-4-en-3-one dehydrogenase [NAD(P)+] activity [GO:0047006], pregnan-21-ol dehydrogenase (NAD+) activity [GO:0047007], pregnan-21-ol dehydrogenase (NADP+) activity [GO:0047008], GO:0047013, 7-beta-hydroxysteroid dehydrogenase (NADP+) activity [GO:0047022], androsterone dehydrogenase [NAD(P)+] activity [GO:0047023], 5-alpha-androstane-3-beta,17-beta-diol dehydrogenase (NADP+) activity [GO:0047024], androstan-3-alpha,17-beta-diol dehydrogenase (NAD+) activity [GO:0047044], 12-beta-hydroxysteroid dehydrogenase (NADP+) activity [GO:0047521], estradiol 17-alpha-dehydrogenase [NAD(P)+] activity [GO:0047881], 11-beta-hydroxysteroid dehydrogenase (NAD+) activity [GO:0070523], 11-beta-hydroxysteroid dehydrogenase (NADP+) activity [GO:0070524], 17-beta-hydroxysteroid dehydrogenase (NADP+) activity [GO:0072582], chenodeoxycholate 7-alpha-dehydrogenase (NAD+) activity [GO:0106281], GO:0106282, ursodeoxycholate 7-beta-dehydrogenase (NAD+) activity [GO:0106283], GO:0140169